{
  "gene_symbol": "PAWR",
  "gene_name": "PRKC apoptosis WT1 regulator protein",
  "gene": "UniProtKB:Q96IZ0",
  "term_label": "apoptotic signaling pathway",
  "term_id": "GO:0097190"
}